{
  "gene": "UniProtKB:P22362",
  "gene_name": "C-C motif chemokine 1",
  "term_id": "GO:0070098",
  "term_label": "chemokine-mediated signaling pathway",
  "gene_symbol": "CCL1"
}